{
  "gene_name": "Immunoglobulin heavy variable 4-31",
  "gene_symbol": "IGHV4-31",
  "term_label": "immunoglobulin mediated immune response",
  "term_id": "GO:0016064",
  "gene": "UniProtKB:P0DP07"
}